regulation of meiotic cell cycle process involved in oocyte maturation [GO:1903538] (biological process) References: PMID:25212395 Sources: GOC:TermGenie, GOC:jz, GO_REF:0000058 Also known as: regulation of meiosis involved in oocyte maturation Relationships: is a type of regulation of cell cycle process [GO:0010564]; is a type of regulation of reproductive process [GO:2000241]; regulates GO:1903537 Subtypes: negative regulation of meiotic cell cycle process involved in oocyte maturation [GO:1904145], positive regulation of meiotic cell cycle process involved in oocyte maturation [GO:1904146] Definition: Any process that modulates the frequency, rate or extent of meiotic cell cycle process involved in oocyte maturation.